protein localization to cleavage furrow rim [GO:1905346] (biological process) Definition: A process in which a protein is transported to, or maintained in, a location within a cleavage furrow rim. References: PMID:27082518 Sources: GOC:TermGenie, GO_REF:0000087 Also known as: protein localisation in cleavage furrow rim, protein localisation to cleavage furrow rim, protein localization in cleavage furrow rim Relationships: is a type of protein localization to cleavage furrow [GO:1905345]